{
  "gene_symbol": "OR8G5",
  "term_id": "GO:0007608",
  "gene": "UniProtKB:Q8NG78",
  "term_label": "sensory perception of smell",
  "gene_name": "Olfactory receptor 8G5"
}